endocardial cushion to mesenchymal transition involved in cardiac skeleton development [GO:0003202] (biological process) Relationships: is a type of endocardial cushion to mesenchymal transition [GO:0090500]; is part of cardiac skeleton development [GO:0003204] Sources: GOC:mtg_heart Definition: A transition where an endocardial cushion cell loses apical/basolateral polarity, severs intercellular adhesive junctions, degrades basement membrane components and becomes a migratory mesenchymal cell that will give rise to the cardiac skeleton.